{
  "gene": "UniProtKB:A6NFC5",
  "gene_name": "Transmembrane protein 235",
  "term_id": "GO:0016324",
  "term_label": "apical plasma membrane",
  "gene_symbol": "TMEM235"
}